{
  "gene_symbol": "NFATC2IP",
  "gene_name": "NFATC2-interacting protein",
  "gene": "UniProtKB:Q8NCF5",
  "term_id": "UNKNOWN:0001",
  "term_label": "Unknown molecular function"
}